nuclear polyadenylation-dependent mRNA catabolic process [GO:0071042] (biological process) Relationships: is a type of GO:0071047 Also known as: nuclear poly(A)-dependent mRNA catabolic process Definition: The chemical reactions and pathways occurring in the nucleus and resulting in the breakdown of a messenger RNA (mRNA) molecule, initiated by the enzymatic addition of a sequence of adenylyl residues (polyadenylation) at the 3' end the target mRNA. References: PMID:15145828, PMID:15828860, PMID:16431988, PMID:17643380, PMID:18000032, PMID:18644474 Sources: GOC:dgf, GOC:krc